{
  "gene_name": "Fractalkine",
  "term_label": "chemokine-mediated signaling pathway",
  "gene": "UniProtKB:P78423",
  "gene_symbol": "CX3CL1",
  "term_id": "GO:0070098"
}